{
  "gene_symbol": "DDX3X",
  "term_id": "GO:0007276",
  "gene_name": "ATP-dependent RNA helicase DDX3X",
  "gene": "UniProtKB:O00571",
  "term_label": "gamete generation"
}